{
  "gene_name": "Sodium bicarbonate cotransporter 3",
  "gene": "UniProtKB:Q9Y6M7",
  "term_label": "plasma membrane",
  "term_id": "GO:0005886",
  "gene_symbol": "SLC4A7"
}